nematode pharyngeal pumping [GO:0043050] (biological process) Relationships: is_a eating behavior [GO:0042755] Regulation: regulated by regulation of nematode pharyngeal pumping [GO:0043051]; negatively regulated by negative regulation of nematode pharyngeal pumping [GO:1903745]; positively regulated by positive regulation of nematode pharyngeal pumping [GO:1903746] Definition: The contraction and relaxation movements of the pharyngeal muscle that mediate feeding in nematodes. References: PMID:2181052 Sources: GOC:cab1 Also known as: pumping behavior